{
  "gene_name": "Histamine N-methyltransferase",
  "term_label": "histamine N-methyltransferase activity",
  "gene_symbol": "HNMT",
  "term_id": "GO:0046539",
  "gene": "UniProtKB:P50135"
}